positive regulation of telomere maintenance via recombination [GO:0032209] (biological process) Definition: Any process that activates or increases the frequency, rate or extent of a recombinational process involved in the maintenance of proper telomeric length. Also known as: up regulation of telomere maintenance via recombination, up-regulation of telomere maintenance via recombination, upregulation of telomere maintenance via recombination, activation of telomere maintenance via recombination, stimulation of telomere maintenance via recombination Sources: GOC:mah Relationships: is a type of positive regulation of telomere maintenance [GO:0032206]; is a type of regulation of telomere maintenance via recombination [GO:0032207]; is a type of positive regulation of mitotic recombination [GO:0045951]; is a type of GO:0072696; positively regulates telomere maintenance via recombination [GO:0000722]